{
  "gene_symbol": "ZNF572",
  "gene": "UniProtKB:Q7Z3I7",
  "term_label": "regulation of cytokine production",
  "gene_name": "Zinc finger protein 572",
  "term_id": "GO:0001817"
}